positive regulation of hemocyte proliferation [GO:0035208] (biological process) Sources: GOC:bf, GOC:mtg_sensu Relationships: is a type of positive regulation of immune system process [GO:0002684]; is a type of positive regulation of cell population proliferation [GO:0008284]; is a type of regulation of hemocyte proliferation [GO:0035206]; RO_0002213 GO:0035172 Also known as: positive regulation of arthropod blood cell proliferation, up regulation of hemocyte proliferation, up-regulation of hemocyte proliferation, upregulation of hemocyte proliferation, activation of hemocyte proliferation, stimulation of hemocyte proliferation Definition: Any process that activates or increases the rate or extent of hemocyte proliferation. Hemocytes are blood cells associated with a hemocoel (the cavity containing most of the major organs of the arthropod body) that are involved in defense and clotting of hemolymph, but not involved in transport of oxygen. An example of this process is found in Drosophila melanogaster.